{
  "gene": "UniProtKB:Q0P651",
  "term_id": "UNKNOWN:0001",
  "term_label": "Unknown molecular function",
  "gene_name": "Protein ABHD18",
  "gene_symbol": "ABHD18"
}